{
  "gene_name": "Tryptophan 5-hydroxylase 2",
  "gene_symbol": "TPH2",
  "term_id": "GO:0004510",
  "gene": "UniProtKB:Q8IWU9",
  "term_label": "tryptophan 5-monooxygenase activity"
}